purine ribonucleoside bisphosphate biosynthetic process [GO:0034036] (biological process) Definition: The chemical reactions and pathways resulting in the formation of a purine ribonucleoside bisphosphate, a compound consisting of a purine base linked to a ribose sugar esterified with one phosphate group attached to each of two different hydroxyl groups on the sugar. Relationships: is a type of ribonucleoside bisphosphate biosynthetic process [GO:0034030]; is a type of GO:0034033; is a type of purine ribonucleoside bisphosphate metabolic process [GO:0034035] Also known as: purine ribonucleoside bisphosphate anabolism, purine ribonucleoside bisphosphate biosynthesis, purine ribonucleoside bisphosphate formation, purine ribonucleoside bisphosphate synthesis Sources: GOC:mah, GOC:pde Subtypes: guanosine tetraphosphate biosynthetic process [GO:0015970], guanosine pentaphosphate biosynthetic process [GO:0015973], GO:0050428